{
  "gene_name": "MOB-like protein phocein",
  "term_label": "cytoplasm",
  "gene_symbol": "MOB4",
  "term_id": "GO:0005737",
  "gene": "UniProtKB:Q9Y3A3"
}